{
  "gene_name": "E3 ubiquitin-protein ligase TRIM52",
  "gene": "UniProtKB:Q96A61",
  "gene_symbol": "TRIM52",
  "term_label": "cytoplasm",
  "term_id": "GO:0005737"
}